{
  "gene": "UniProtKB:Q9C0D0",
  "term_id": "GO:0003779",
  "term_label": "actin binding",
  "gene_name": "Phosphatase and actin regulator 1",
  "gene_symbol": "PHACTR1"
}